{
  "term_label": "bone development",
  "gene_symbol": "TGM2",
  "term_id": "GO:0060348",
  "gene": "UniProtKB:P21980",
  "gene_name": "Protein-glutamine gamma-glutamyltransferase 2"
}